{
  "gene": "UniProtKB:Q8IZR5",
  "gene_symbol": "CMTM4",
  "gene_name": "CKLF-like MARVEL transmembrane domain-containing protein 4",
  "term_id": "UNKNOWN:0002",
  "term_label": "Unknown biological process"
}